dense core granule transport [GO:1901950] (biological process) Relationships: is a type of cytosolic transport [GO:0016482]; is_a dense core granule localization [GO:0032253]; is_a GO:0051650 References: PMID:23358451 Sources: GOC:TermGenie, GOC:kmv Definition: The directed movement a dense core granule within a cell. Also known as: dense core vesicle transport Note: goslim_synapse Subtypes: dense core granule cytoskeletal transport [GO:0099519] Regulation: regulated by regulation of dense core granule transport [GO:1904809]; negatively regulated by negative regulation of dense core granule transport [GO:1904810]; positively regulated by positive regulation of dense core granule transport [GO:1904811]